{
  "gene": "UniProtKB:Q8NC69",
  "term_id": "UNKNOWN:0003",
  "gene_name": "BTB_POZ domain-containing protein KCTD6",
  "term_label": "Unknown cellular component",
  "gene_symbol": "KCTD6"
}